{
  "term_id": "GO:0003692",
  "gene": "UniProtKB:Q9H171",
  "term_label": "left-handed Z-DNA binding",
  "gene_name": "Z-DNA-binding protein 1",
  "gene_symbol": "ZBP1"
}